{
  "term_label": "mRNA 3'-UTR binding",
  "gene": "UniProtKB:P0CB38",
  "term_id": "GO:0003730",
  "gene_name": "Polyadenylate-binding protein 4-like",
  "gene_symbol": "PABPC4L"
}